{
  "term_label": "lysosome organization",
  "gene_name": "Ceroid-lipofuscinosis neuronal protein 5",
  "term_id": "GO:0007040",
  "gene": "UniProtKB:O75503",
  "gene_symbol": "CLN5"
}